{
  "gene_symbol": "SMCO4",
  "term_label": "Unknown biological process",
  "gene": "UniProtKB:Q9NRQ5",
  "term_id": "UNKNOWN:0002",
  "gene_name": "Single-pass membrane and coiled-coil domain-containing protein 4"
}